{
  "term_label": "Unknown biological process",
  "gene_name": "Guanylate cyclase activator 2B",
  "term_id": "UNKNOWN:0002",
  "gene_symbol": "GUCA2B",
  "gene": "UniProtKB:Q16661"
}